{
  "gene_symbol": "DPP8",
  "gene": "UniProtKB:Q6V1X1",
  "term_label": "proteolysis",
  "gene_name": "Dipeptidyl peptidase 8",
  "term_id": "GO:0006508"
}